{
  "gene": "UniProtKB:Q9NVU7",
  "gene_symbol": "SDAD1",
  "term_label": "Unknown molecular function",
  "gene_name": "Protein SDA1 homolog",
  "term_id": "UNKNOWN:0001"
}